P-type sodium transporter activity [GO:0008554] (molecular function) Also known as: Na(+)-exporting ATPase activity, Na(+)-transporting ATPase activity, Na+-exporting ATPase activity, Na+-transporting ATPase activity, sodium transport ATPase activity, sodium-exporting ATPase activity, sodium exporting ATPase activity, phosphorylative mechanism, sodium transmembrane transporter activity, phosphorylative mechanism, sodium-exporting ATPase activity, phosphorylative mechanism, sodium-translocating P-type ATPase activity References: PMID:9224683 Relationships: is a type of sodium ion transmembrane transporter activity [GO:0015081]; is a type of P-type ion transporter activity [GO:0015662]; is a type of ATPase-coupled monoatomic cation transmembrane transporter activity [GO:0019829] Subtypes: P-type sodium:potassium-exchanging transporter activity [GO:0005391] Note: Note that RHEA:14633 represents both the ABC and the P-type sodium transporters. Definition: Enables the transfer of a solute or solutes from one side of a membrane to the other according to the reaction: ATP + H2O + Na+(in) = ADP + phosphate + Na+(out); by a phosphorylative mechanism.